{
  "gene": "UniProtKB:P02775",
  "term_label": "CXCR chemokine receptor binding",
  "gene_symbol": "PPBP",
  "term_id": "GO:0045236",
  "gene_name": "Platelet basic protein"
}